oxidoreductase activity, acting on the CH-NH2 group of donors, disulfide as acceptor [GO:0016642] (molecular function) Relationships: is a type of oxidoreductase activity, acting on the CH-NH2 group of donors [GO:0016638] Sources: GOC:ai Definition: Catalysis of an oxidation-reduction (redox) reaction in which a CH-NH2 group acts as a hydrogen or electron donor and reduces a disulfide group. Also known as: oxidoreductase activity, acting on the CH-NH2 group of donors, disulphide as acceptor Subtypes: glycine dehydrogenase (decarboxylating) activity [GO:0004375]